{
  "term_id": "GO:0031080",
  "term_label": "nuclear pore outer ring",
  "gene_name": "Nucleoporin Nup43",
  "gene_symbol": "NUP43",
  "gene": "UniProtKB:Q8NFH3"
}